{
  "term_id": "GO:0008381",
  "gene_symbol": "TMC4",
  "gene_name": "Transmembrane channel-like protein 4",
  "gene": "UniProtKB:Q7Z404",
  "term_label": "mechanosensitive monoatomic ion channel activity"
}